{
  "term_label": "hippo signaling",
  "gene": "UniProtKB:O95835",
  "gene_symbol": "LATS1",
  "gene_name": "Serine_threonine-protein kinase LATS1",
  "term_id": "GO:0035329"
}